{
  "gene_name": "Leukemia-associated protein 1",
  "term_id": "UNKNOWN:0003",
  "gene_symbol": "DLEU1",
  "gene": "UniProtKB:O43261",
  "term_label": "Unknown cellular component"
}